indole glucosinolate metabolic process [GO:0042343] (biological process) Definition: The chemical reactions and pathways resulting in the formation of indole glucosinolates. Glucosinolates are sulfur-containing compounds that have a common structure linked to an R group derived from tryptophan; indoles are biologically active substances based on 2,3-benzopyrrole, formed during the catabolism of tryptophan. Sources: GOC:curators Also known as: indole glucosinolate metabolism Relationships: is a type of glucosinolate metabolic process [GO:0019760]; is a type of GO:0042430 Subtypes: indole glucosinolate biosynthetic process [GO:0009759], indole glucosinolate catabolic process [GO:0042344]